{
  "term_label": "RNA polymerase II cis-regulatory region sequence-specific DNA binding",
  "gene_symbol": "MECOM",
  "gene_name": "Histone-lysine N-methyltransferase MECOM",
  "term_id": "GO:0000978",
  "gene": "UniProtKB:Q03112"
}